{
  "term_label": "response to exogenous dsRNA",
  "gene": "UniProtKB:P01567",
  "gene_name": "Interferon alpha-7",
  "gene_symbol": "IFNA7",
  "term_id": "GO:0043330"
}